{
  "gene": "UniProtKB:Q12788",
  "term_id": "GO:0030686",
  "term_label": "90S preribosome",
  "gene_name": "Transducin beta-like protein 3",
  "gene_symbol": "TBL3"
}